galactosylacylglycerol O-acyltransferase activity [GO:0047175] (molecular function) Definition: Catalysis of the reaction: sn-3-D-galactosyl-sn-2-acylglycerol + acyl-[acyl-carrier protein] = D-galactosyldiacylglycerol + [acyl-carrier protein]. Sources: EC:2.3.1.141, MetaCyc:2.3.1.141-RXN Relationships: is a type of O-acyltransferase activity [GO:0008374] Also known as: acyl-ACP:lyso-MGDG acyltransferase activity, acyl-acyl-carrier protein: lysomonogalactosyldiacylglycerol acyltransferase activity, acyl-acyl-carrier-protein:D-galactosylacylglycerol O-acyltransferase activity